{
  "gene_symbol": "CRISP1",
  "term_label": "Unknown biological process",
  "term_id": "UNKNOWN:0002",
  "gene": "UniProtKB:P54107",
  "gene_name": "Cysteine-rich secretory protein 1"
}